regulation of sodium ion transmembrane transport [GO:1902305] (biological process) Relationships: is a type of regulation of sodium ion transport [GO:0002028]; is a type of regulation of monoatomic cation transmembrane transport [GO:1904062]; regulates GO:0035725 References: PMID:18591664 Sources: GOC:BHF, GOC:TermGenie, GOC:mtg_cardiac_conduct_nov11, GOC:rl Also known as: regulation of sodium ion membrane transport Subtypes: negative regulation of sodium ion transmembrane transport [GO:1902306], GO:1902307, GO:1903276, regulation of sodium ion import across plasma membrane [GO:1903782], regulation of sodium ion transmembrane transporter activity [GO:2000649] Definition: Any process that modulates the frequency, rate or extent of sodium ion transmembrane transport.